L-tryptophan catabolic process to kynurenine [GO:0019441] (biological process) Definition: The chemical reactions and pathways resulting in the breakdown of L-tryptophan into other compounds, including kynurenine. Sources: GOC:go_curators Also known as: tryptophan breakdown to kynurenine, tryptophan catabolic process to kynurenine, tryptophan degradation to kynurenine Relationships: is a type of L-tryptophan catabolic process [GO:0006569]; is_a kynurenine metabolic process [GO:0070189]